paranode region of axon [GO:0033270] (cellular component) Relationships: is a type of cellular anatomical structure [GO:0110165]; is part of main axon [GO:0044304] Sources: GOC:mah, GOC:mh, NIF_Subcellular:sao936144858 Definition: An axon part that is located adjacent to the nodes of Ranvier and surrounded by lateral loop portions of myelin sheath. Also known as: paranode